{
  "gene_symbol": "ZNF534",
  "gene_name": "Zinc finger protein 534",
  "term_id": "GO:0005634",
  "gene": "UniProtKB:Q76KX8",
  "term_label": "nucleus"
}